basic amino acid transmembrane transporter activity [GO:0015174] (molecular function) Definition: Enables the transfer of basic amino acids from one side of a membrane to the other. Basic amino acids have side chains with a positive charge at pH 7.3. Sources: GOC:ai, GOC:mtg_transport, ISBN:0815340729 Also known as: basic amino acid transporter activity, basic amino acid permease activity, cationic amino acid transmembrane transporter activity Relationships: is a type of amino acid transmembrane transporter activity [GO:0015171]; is part of basic amino acid transmembrane transport [GO:1990822] Subtypes: high-affinity basic amino acid transmembrane transporter activity [GO:0005287], L-histidine transmembrane transporter activity [GO:0005290], L-lysine transmembrane transporter activity [GO:0015189], GO:0061459, GO:0097625, broad specificity neutral L-amino acid:basic L-amino acid antiporter activity [GO:0180009]